hydroxyectoine binding [GO:0033295] (molecular function) Definition: Binding to hydroxyectoine. Sources: GOC:mlg Relationships: is a type of GO:0033293; is a type of GO:0043178; is a type of quaternary ammonium group binding [GO:0050997]; is a type of heterocyclic compound binding [GO:1901363]